carbon dioxide transmembrane transport [GO:0035378] (biological process) Relationships: is a type of carbon dioxide transport [GO:0015670]; is a type of transmembrane transport [GO:0055085] Definition: The process in which carbon dioxide (CO2) is transported across a membrane. Also known as: carbon dioxide membrane transport Sources: GOC:yaf Note: Note that this term is not intended for use in annotating lateral movement within membranes.